{
  "gene": "UniProtKB:P11488",
  "term_label": "cytoplasm",
  "gene_name": "Guanine nucleotide-binding protein G(t) subunit alpha-1",
  "term_id": "GO:0005737",
  "gene_symbol": "GNAT1"
}